{
  "gene_symbol": "H2BC13",
  "gene": "UniProtKB:Q99880",
  "term_label": "antimicrobial humoral immune response mediated by antimicrobial peptide",
  "gene_name": "Histone H2B type 1-L",
  "term_id": "GO:0061844"
}